{
  "term_label": "regulation of signal transduction",
  "gene_symbol": "GUCA1C",
  "gene_name": "Guanylyl cyclase-activating protein 3",
  "gene": "UniProtKB:O95843",
  "term_id": "GO:0009966"
}